cellular response to methylamine [GO:0036256] (biological process) Relationships: is a type of GO:0036255; is a type of GO:0071418 Definition: Any process that results in a change in state or activity of a cell (in terms of movement, secretion, enzyme production, gene expression, etc.) as a result of a methylamine stimulus. Sources: GOC:mah